positive regulation of appressorium formation [GO:0075018] (BP) Definition: Any process that activates or increases the frequency, rate or extent of symbiont appressorium formation. Relationships: is a type of positive regulation of developmental process [GO:0051094]; is a type of regulation of appressorium formation [GO:0075017]; positively regulates appressorium formation [GO:0075016] Sources: GOC:pamgo_curators Also known as: positive regulation of appressorium formation on or near host Note: Note that this term should not be used to annotate gene products of the host. It should only be used to annotate those gene products from the symbiont involved in this process.